{
  "gene_name": "Phosphoinositide-interacting protein",
  "term_id": "GO:0051930",
  "term_label": "regulation of sensory perception of pain",
  "gene": "UniProtKB:P0C851",
  "gene_symbol": "PIRT"
}